{
  "gene_symbol": "FAM50A",
  "term_id": "GO:0006325",
  "gene_name": "Protein FAM50A",
  "gene": "UniProtKB:Q14320",
  "term_label": "chromatin organization"
}